UDP-N-acetyl-alpha-D-quinovosamine dehydrogenase activity [GO:0102538] (molecular function) Relationships: is_a oxidoreductase activity, acting on the CH-OH group of donors, NAD or NADP as acceptor [GO:0016616] References: PMID:10627048, PMID:24817117 Sources: GOC:pz Definition: Catalysis of the reaction: UDP-N-acetyl-alpha-D-quinovosamine + NAD(P) = UDP-2-acetamido-4-dehydro-2,6-dideoxy-beta-D-glucose + H+ + NAD(P)H.